{
  "term_id": "GO:0031013",
  "gene_name": "Troponin T, cardiac muscle",
  "term_label": "troponin I binding",
  "gene": "UniProtKB:P45379",
  "gene_symbol": "TNNT2"
}